{
  "gene_name": "Protein EOLA1",
  "gene": "UniProtKB:Q8TE69",
  "term_label": "Unknown cellular component",
  "term_id": "UNKNOWN:0003",
  "gene_symbol": "EOLA1"
}